{
  "gene_symbol": "MOG",
  "term_label": "signaling receptor binding",
  "gene": "UniProtKB:Q16653",
  "gene_name": "Myelin-oligodendrocyte glycoprotein",
  "term_id": "GO:0005102"
}